{
  "term_id": "GO:0055003",
  "gene_name": "Telethonin",
  "gene": "UniProtKB:O15273",
  "term_label": "cardiac myofibril assembly",
  "gene_symbol": "TCAP"
}